{
  "term_id": "GO:0047499",
  "term_label": "calcium-independent phospholipase A2 activity",
  "gene_name": "Phospholipase A2 group XV",
  "gene_symbol": "PLA2G15",
  "gene": "UniProtKB:Q8NCC3"
}